{
  "gene": "UniProtKB:P62820",
  "gene_name": "Ras-related protein Rab-1A",
  "gene_symbol": "RAB1A",
  "term_label": "intracellular protein transport",
  "term_id": "GO:0006886"
}